{
  "gene": "UniProtKB:P25774",
  "term_id": "GO:0005764",
  "gene_symbol": "CTSS",
  "gene_name": "Cathepsin S",
  "term_label": "lysosome"
}